{
  "gene": "UniProtKB:P11465",
  "term_label": "Unknown molecular function",
  "gene_name": "Pregnancy-specific beta-1-glycoprotein 2",
  "term_id": "UNKNOWN:0001",
  "gene_symbol": "PSG2"
}